{
  "gene_name": "Beta-defensin 123",
  "gene": "UniProtKB:Q8N688",
  "gene_symbol": "DEFB123",
  "term_id": "UNKNOWN:0003",
  "term_label": "Unknown cellular component"
}